{
  "gene": "UniProtKB:P0DPB6",
  "term_label": "RNA polymerase III complex",
  "gene_symbol": "POLR1D",
  "gene_name": "DNA-directed RNA polymerases I and III subunit RPAC2",
  "term_id": "GO:0005666"
}